{
  "gene_name": "Tumor necrosis factor receptor superfamily member 11B",
  "term_label": "Unknown biological process",
  "gene_symbol": "TNFRSF11B",
  "term_id": "UNKNOWN:0002",
  "gene": "UniProtKB:O00300"
}